{
  "term_id": "GO:0005654",
  "term_label": "nucleoplasm",
  "gene_name": "E3 ubiquitin-protein ligase TRIM22",
  "gene_symbol": "TRIM22",
  "gene": "UniProtKB:Q8IYM9"
}